{
  "gene_name": "Receptor-interacting serine_threonine-protein kinase 4",
  "term_label": "cytoplasm",
  "gene_symbol": "RIPK4",
  "gene": "UniProtKB:P57078",
  "term_id": "GO:0005737"
}